deoxycytidine metabolic process [GO:0046092] (biological process) Sources: GOC:go_curators Relationships: is a type of GO:0046125 Subtypes: deoxycytidine catabolic process [GO:0006217], GO:0046093 Definition: The chemical reactions and pathways involving deoxycytidine, 2-deoxyribosylcytosine, one of the four major nucleosides of DNA. Also known as: deoxycytidine metabolism